{
  "term_id": "UNKNOWN:0002",
  "gene_name": "Uncharacterized protein C16orf74",
  "gene": "UniProtKB:Q96GX8",
  "term_label": "Unknown biological process",
  "gene_symbol": "C16orf74"
}